encysted zoospore germination [GO:0075226] (biological process) Sources: GOC:pamgo_curators Also known as: encysted zoospore germination on or near host Regulation: regulated by regulation of encysted zoospore germination [GO:0075227]; RO_0002213 by GO:0075228; RO_0002212 by negative regulation of encysted zoospore germination [GO:0075229] Relationships: is a type of spore germination [GO:0009847] Note: Note that this term should not be used to annotate gene products of the host. It should only be used to annotate those gene products from the symbiont involved in this process. Definition: The physiological, developmental and morphological changes that occur in an encysted zoospore, that germinates by developing a germ tube that may penetrate the host directly or indirectly through an appressorium. An encysted zoospore is a zoospore which has shed its flagellum and whose membrane has fused to form a walled cyst. The host is defined as the larger of the organisms involved in a symbiotic interaction.